{
  "gene": "UniProtKB:Q9UM11",
  "gene_name": "Fizzy-related protein homolog",
  "gene_symbol": "FZR1",
  "term_label": "positive regulation of anaphase-promoting complex-dependent catabolic process",
  "term_id": "GO:1905786"
}